{
  "term_label": "Unknown molecular function",
  "gene_name": "Pregnancy-specific beta-1-glycoprotein 3",
  "term_id": "UNKNOWN:0001",
  "gene": "UniProtKB:Q16557",
  "gene_symbol": "PSG3"
}